{
  "term_id": "GO:0031167",
  "term_label": "rRNA methylation",
  "gene_name": "Dimethyladenosine transferase 1, mitochondrial",
  "gene": "UniProtKB:Q8WVM0",
  "gene_symbol": "TFB1M"
}